{
  "term_label": "response to lipopolysaccharide",
  "term_id": "GO:0032496",
  "gene_symbol": "S100A14",
  "gene": "UniProtKB:Q9HCY8",
  "gene_name": "Protein S100-A14"
}